generation of ovulation cycle rhythm [GO:0060112] (biological process) Relationships: is_a GO:0022602 Definition: The process which controls the timing of the type of sexual cycle seen in female mammals. Sources: GOC:dph Also known as: generation of estrus cycle rhythm, generation of oestrus cycle rhythm, generation of menstrual cycle rhythm